translation repressor activity, non-nucleic acid binding [GO:0000901] (molecular function) Definition: Antagonizes the ribosome-mediated translation of mRNA into a polypeptide but does not bind directly to nucleic acid. Sources: GOC:clt Relationships: is a type of translation repressor activity [GO:0030371]